interleukin-13-mediated signaling pathway [GO:0035772] (biological process) Relationships: is a type of cytokine-mediated signaling pathway [GO:0019221]; is part of cellular response to interleukin-13 [GO:0035963] Definition: The series of molecular signals initiated by interleukin-13 binding to its receptor on the surface of a target cell, and ending with the regulation of a downstream cellular process, e.g. transcription. Also known as: IL-13-mediated signaling pathway, interleukin-13-mediated signalling pathway Sources: GOC:BHF, GOC:signaling